{
  "gene": "UniProtKB:O94989",
  "gene_name": "Rho guanine nucleotide exchange factor 15",
  "term_label": "guanyl-nucleotide exchange factor activity",
  "gene_symbol": "ARHGEF15",
  "term_id": "GO:0005085"
}